{
  "term_label": "nucleus",
  "term_id": "GO:0005634",
  "gene_symbol": "HES5",
  "gene": "UniProtKB:Q5TA89",
  "gene_name": "Transcription factor HES-5"
}